{
  "gene_name": "Fructose-bisphosphate aldolase B",
  "term_id": "GO:0005829",
  "term_label": "cytosol",
  "gene_symbol": "ALDOB",
  "gene": "UniProtKB:P05062"
}